{
  "term_label": "histone deacetylase binding",
  "gene_name": "Metastasis-associated protein MTA3",
  "term_id": "GO:0042826",
  "gene": "UniProtKB:Q9BTC8",
  "gene_symbol": "MTA3"
}